response to misfolded protein [GO:0051788] (biological process) Subtypes: detection of misfolded protein [GO:0002236], cellular response to misfolded protein [GO:0071218] Relationships: is_a response to topologically incorrect protein [GO:0035966] Definition: Any process that results in a change in state or activity of a cell or an organism (in terms of movement, secretion, enzyme production, gene expression, etc.) as a result of a misfolded protein stimulus. Sources: GOC:go_curators